pronephric nephron tubule morphogenesis [GO:0039008] (biological process) Sources: GOC:mtg_kidney_jan10, ZFA:00001558 Subtypes: pronephric proximal tubule morphogenesis [GO:0039011], pronephric distal tubule morphogenesis [GO:0039013] Relationships: is_a nephron tubule morphogenesis [GO:0072078]; BFO_0000050 pronephric nephron morphogenesis [GO:0039007]; is part of pronephric nephron tubule development [GO:0039020] Definition: The process in which the anatomical structures of a pronephric nephron tubule are generated and organized from an epithelium. A pronephric nephron tubule is an epithelial tube that is part of the pronephric nephron.